{
  "gene_name": "Glutamine and serine-rich protein 1",
  "term_label": "Unknown cellular component",
  "gene_symbol": "QSER1",
  "term_id": "UNKNOWN:0003",
  "gene": "UniProtKB:Q2KHR3"
}